{
  "term_label": "RNA polymerase II transcription regulatory region sequence-specific DNA binding",
  "gene_name": "Neuronal PAS domain-containing protein 1",
  "gene": "UniProtKB:Q99742",
  "term_id": "GO:0000977",
  "gene_symbol": "NPAS1"
}